{
  "term_label": "stretch-activated, monoatomic cation-selective, calcium channel activity",
  "gene_symbol": "NALF1",
  "term_id": "GO:0015275",
  "gene_name": "NALCN channel auxiliary factor 1",
  "gene": "UniProtKB:B1AL88"
}